{
  "gene_symbol": "OTOG",
  "term_id": "GO:0005201",
  "gene": "UniProtKB:Q6ZRI0",
  "gene_name": "Otogelin",
  "term_label": "extracellular matrix structural constituent"
}